negative regulation of cornification [GO:1905716] (biological process) Also known as: down regulation of cornification, down-regulation of cornification, downregulation of cornification, inhibition of cornification Definition: Any process that stops, prevents or reduces the frequency, rate or extent of cornification. References: PMID:26014679 Sources: GOC:TermGenie, GO_REF:0000058 Relationships: is a type of negative regulation of programmed cell death [GO:0043069]; is a type of regulation of cornification [GO:1905715]; negatively regulates cornification [GO:0070268]